{
  "term_label": "Notch signaling pathway",
  "gene_symbol": "HELT",
  "gene_name": "Hairy and enhancer of split-related protein HELT",
  "gene": "UniProtKB:A6NFD8",
  "term_id": "GO:0007219"
}